netrin receptor activity [GO:0005042] (molecular function) Subtypes: netrin receptor activity involved in chemorepulsion [GO:0005043], netrin receptor activity involved in chemoattraction [GO:0038006] Definition: Combining with a netrin signal and transmitting the signal from one side of the membrane to the other to initiate a change in cell activity. References: PMID:15960985 Sources: GOC:dph, GOC:signaling Relationships: is a type of GO:0004888; is part of netrin-activated signaling pathway [GO:0038007]